{
  "term_label": "Unknown cellular component",
  "gene_name": "Serine_threonine-protein kinase 19",
  "gene_symbol": "STK19",
  "gene": "UniProtKB:P49842",
  "term_id": "UNKNOWN:0003"
}